integument-mediated background adaptation [GO:0120304] (biological process) Relationships: is a type of background adaptation [GO:0120302] Definition: Any process in which an organism changes its pigmentation (lightening in response to a brighter environment or darkening in response to a dimmer environment) in response to a change in light intensity detected by light sensitive cells in the integument. References: PMID:29239123, PMID:32898924 Sources: GOC:cvs, GOC:krc